{
  "gene_name": "Polyhomeotic-like protein 1",
  "gene": "UniProtKB:P78364",
  "term_label": "chromatin binding",
  "term_id": "GO:0003682",
  "gene_symbol": "PHC1"
}